{
  "term_id": "GO:0005634",
  "term_label": "nucleus",
  "gene": "UniProtKB:P17066",
  "gene_symbol": "HSPA6",
  "gene_name": "Heat shock 70 kDa protein 6"
}